{
  "term_id": "GO:1903804",
  "gene": "UniProtKB:Q9Y345",
  "term_label": "glycine import across plasma membrane",
  "gene_name": "Sodium- and chloride-dependent glycine transporter 2",
  "gene_symbol": "SLC6A5"
}